amyloid fibril formation [GO:1990000] (biological process) Also known as: amyloid fibril assembly, amyloid structure assembly, amyloid structure formation Definition: The generation of amyloid fibrils, insoluble fibrous protein aggregates exhibiting beta sheet structure, from proteins. Note: Although deposition of amyloid fibrils is associated with diseases, e.g. Alzheimer's disease, amyloid formation is a normal process. Disease occurs when the balance between amyloid formation and clearance is disrupted (reviewed e.g. in PMID:29654159 and PMID:28937655). An example of a normal amyloid complex is composed of human RIP1 and RIP3 kinases (PMID:22817896). Relationships: is a type of GO:0019538; is a type of supramolecular fiber organization [GO:0097435] Regulation: regulated by regulation of amyloid fibril formation [GO:1905906]; negatively regulated by negative regulation of amyloid fibril formation [GO:1905907]; positively regulated by positive regulation of amyloid fibril formation [GO:1905908] References: PMID:21148556, PMID:22817896, PMID:28937655, PMID:29654159 Sources: GOC:cvs, GOC:jj, GOC:ppm, GOC:sj